{
  "gene": "UniProtKB:Q86SE9",
  "term_label": "Unknown molecular function",
  "term_id": "UNKNOWN:0001",
  "gene_name": "Polycomb group RING finger protein 5",
  "gene_symbol": "PCGF5"
}